deoxyribose-phosphate aldolase activity [GO:0004139] (molecular function) Also known as: 2-deoxy-D-ribose-5-phosphate acetaldehyde-lyase (D-glyceraldehyde-3-phosphate-forming), 2-deoxy-D-ribose-5-phosphate acetaldehyde-lyase activity, 2-deoxyribose-5-phosphate aldolase activity, deoxyriboaldolase activity, deoxyribose-5-phosphate aldolase activity, phosphodeoxyriboaldolase activity Definition: Catalysis of the reaction: 2-deoxy-D-ribose 5-phosphate = D-glyceraldehyde 3-phosphate + acetaldehyde. Sources: EC:4.1.2.4, RHEA:12821 Relationships: is a type of aldehyde-lyase activity [GO:0016832]